regulation of centriole-centriole cohesion [GO:0030997] (biological process) Relationships: is a type of regulation of cell cycle process [GO:0010564]; is part of GO:0007098; RO_0002211 GO:0010457 References: PMID:11076968 Subtypes: negative regulation of centriole-centriole cohesion [GO:1903126], positive regulation of centriole-centriole cohesion [GO:1903127] Definition: Any process that modulates the extent to which the two centrioles within a centrosome remain tightly paired; may be mediated by the assembly and disassembly of a proteinaceous linker.